{
  "gene_symbol": "GAGE13",
  "gene": "UniProtKB:Q4V321",
  "term_label": "Unknown biological process",
  "gene_name": "G antigen 13",
  "term_id": "UNKNOWN:0002"
}